{
  "gene_name": "ORM1-like protein 2",
  "term_id": "UNKNOWN:0001",
  "gene": "UniProtKB:Q53FV1",
  "gene_symbol": "ORMDL2",
  "term_label": "Unknown molecular function"
}